negative regulation of timing of anagen [GO:0051886] (biological process) Sources: GOC:ai, GOC:pr Relationships: is a type of GO:0048817; is a type of regulation of timing of anagen [GO:0051884]; negatively regulates anagen [GO:0042640] Also known as: inhibition of anagen, down regulation of anagen, down-regulation of anagen, downregulation of anagen, negative regulation of anagen Definition: Any process that stops, prevents, or reduces the frequency, rate or extent of timing of anagen, the growth phase of the hair cycle.